{
  "gene_name": "Uncharacterized protein ZSWIM9",
  "term_id": "UNKNOWN:0002",
  "gene": "UniProtKB:Q86XI8",
  "term_label": "Unknown biological process",
  "gene_symbol": "ZSWIM9"
}